{
  "gene": "UniProtKB:A0A5F9ZH02",
  "term_id": "UNKNOWN:0001",
  "term_label": "Unknown molecular function",
  "gene_name": "Small integral membrane protein 42",
  "gene_symbol": "SMIM42"
}